{
  "gene_symbol": "CENPH",
  "term_label": "chromosome segregation",
  "gene": "UniProtKB:Q9H3R5",
  "term_id": "GO:0007059",
  "gene_name": "Centromere protein H"
}